{
  "gene_name": "Ubiquilin-2",
  "gene": "UniProtKB:Q9UHD9",
  "term_id": "GO:0005829",
  "term_label": "cytosol",
  "gene_symbol": "UBQLN2"
}